{
  "gene_symbol": "LMAN1L",
  "term_id": "GO:0000139",
  "gene": "UniProtKB:Q9HAT1",
  "term_label": "Golgi membrane",
  "gene_name": "Protein ERGIC-53-like"
}